small intestine smooth muscle contraction [GO:1990770] (biological process) References: PMID:11991626 Regulation: regulated by regulation of small intestine smooth muscle contraction [GO:1904347]; negatively regulated by negative regulation of small intestine smooth muscle contraction [GO:1904348]; positively regulated by positive regulation of small intestine smooth muscle contraction [GO:1904349] Definition: A process in which force is generated within smooth muscle tissue, resulting in a change in muscle geometry in the intestine between the stomach and the large intestine. Relationships: is a type of GO:0006939; is part of intestine smooth muscle contraction [GO:0014827]